{
  "term_label": "Unknown biological process",
  "term_id": "UNKNOWN:0002",
  "gene_symbol": "TRDJ3",
  "gene": "UniProtKB:A0A075B6W1",
  "gene_name": "T cell receptor delta joining 3 (Fragment)"
}